{
  "gene_symbol": "NR2E3",
  "gene": "UniProtKB:Q9Y5X4",
  "term_id": "GO:0030182",
  "term_label": "neuron differentiation",
  "gene_name": "Photoreceptor-specific nuclear receptor"
}